{
  "term_id": "GO:0009966",
  "gene_symbol": "KCNIP3",
  "gene_name": "Calsenilin",
  "gene": "UniProtKB:Q9Y2W7",
  "term_label": "regulation of signal transduction"
}